polyphosphate catabolic process [GO:0006798] (biological process) Definition: The chemical reactions and pathways resulting in the breakdown of a polyphosphate, the anion or salt of polyphosphoric acid. Sources: GOC:go_curators, ISBN:0198506732 Also known as: polyphosphate breakdown, polyphosphate catabolism, polyphosphate degradation Relationships: is a type of polyphosphate metabolic process [GO:0006797]; is_a GO:0009056